{
  "gene": "UniProtKB:O75716",
  "term_label": "Unknown biological process",
  "gene_symbol": "STK16",
  "term_id": "UNKNOWN:0002",
  "gene_name": "Serine_threonine-protein kinase 16"
}